{
  "term_id": "GO:0035082",
  "gene": "UniProtKB:Q6NUN7",
  "gene_name": "Jhy protein homolog",
  "term_label": "axoneme assembly",
  "gene_symbol": "JHY"
}